{
  "gene": "UniProtKB:Q5SYB0",
  "term_label": "cell cortex",
  "gene_name": "FERM and PDZ domain-containing protein 1",
  "term_id": "GO:0005938",
  "gene_symbol": "FRMPD1"
}